{
  "gene": "UniProtKB:Q9Y6M4",
  "gene_name": "Casein kinase I isoform gamma-3",
  "gene_symbol": "CSNK1G3",
  "term_id": "GO:0007165",
  "term_label": "signal transduction"
}